{
  "term_id": "GO:0000981",
  "gene": "UniProtKB:Q5CZA5",
  "gene_name": "Zinc finger protein 805",
  "term_label": "DNA-binding transcription factor activity, RNA polymerase II-specific",
  "gene_symbol": "ZNF805"
}